{
  "term_label": "U1 snRNP",
  "term_id": "GO:0005685",
  "gene": "UniProtKB:P62318",
  "gene_symbol": "SNRPD3",
  "gene_name": "Small nuclear ribonucleoprotein Sm D3"
}